{
  "gene_name": "Small conductance calcium-activated potassium channel protein 1",
  "gene_symbol": "KCNN1",
  "term_label": "potassium ion transmembrane transport",
  "gene": "UniProtKB:Q92952",
  "term_id": "GO:0071805"
}